{
  "gene": "UniProtKB:P61088",
  "gene_symbol": "UBE2N",
  "term_id": "GO:0070534",
  "gene_name": "Ubiquitin-conjugating enzyme E2 N",
  "term_label": "protein K63-linked ubiquitination"
}